{
  "term_label": "Unknown cellular component",
  "gene_name": "Chondroitin sulfate N-acetylgalactosaminyltransferase 2",
  "gene_symbol": "CSGALNACT2",
  "term_id": "UNKNOWN:0003",
  "gene": "UniProtKB:Q8N6G5"
}